{
  "gene_symbol": "INSIG2",
  "term_id": "GO:0036316",
  "gene": "UniProtKB:Q9Y5U4",
  "term_label": "SREBP-SCAP complex retention in endoplasmic reticulum",
  "gene_name": "Insulin-induced gene 2 protein"
}